host extracellular space [GO:0043655] (cellular component) Sources: GOC:cc Relationships: is a type of host cellular component [GO:0018995] Definition: The space within a host but external to the plasma membrane of host cells, e.g. within host bloodstream. Also known as: extracellular space of host